cellularization [GO:0007349] (BP) Definition: The separation of a multi-nucleate cell or syncytium into individual cells. An example of this is found in Drosophila melanogaster embryo development. Sources: GOC:go_curators, GOC:mtg_sensu, ISBN:0716731363 Relationships: is a type of anatomical structure formation involved in morphogenesis [GO:0048646]; BFO_0000050 multicellular organism development [GO:0007275] Subtypes: pole cell formation [GO:0007279], sperm individualization [GO:0007291], embryo sac cellularization [GO:0009558], endosperm cellularization [GO:0010342], syncytial embryo cellularization [GO:0110069]